{
  "term_label": "positive regulation of T cell activation",
  "gene_name": "HLA class II histocompatibility antigen, DRB1 beta chain",
  "gene": "UniProtKB:P01911",
  "term_id": "GO:0050870",
  "gene_symbol": "HLA-DRB1"
}